{
  "gene_name": "Cell division cycle protein 23 homolog",
  "gene": "UniProtKB:Q9UJX2",
  "term_id": "GO:0045842",
  "gene_symbol": "CDC23",
  "term_label": "positive regulation of mitotic metaphase/anaphase transition"
}